{
  "term_id": "GO:0005813",
  "gene_symbol": "XRCC2",
  "gene_name": "DNA repair protein XRCC2",
  "gene": "UniProtKB:O43543",
  "term_label": "centrosome"
}